{
  "term_id": "UNKNOWN:0003",
  "term_label": "Unknown cellular component",
  "gene_symbol": "PLCB4",
  "gene_name": "1-phosphatidylinositol 4,5-bisphosphate phosphodiesterase beta-4",
  "gene": "UniProtKB:Q15147"
}